{
  "gene": "UniProtKB:P20073",
  "term_id": "GO:0001786",
  "gene_symbol": "ANXA7",
  "term_label": "phosphatidylserine binding",
  "gene_name": "Annexin A7"
}